{
  "term_label": "L-aspartate:2-oxoglutarate aminotransferase activity",
  "gene_symbol": "GOT2",
  "term_id": "GO:0004069",
  "gene": "UniProtKB:P00505",
  "gene_name": "Aspartate aminotransferase, mitochondrial"
}